BLOC-2 complex binding [GO:0036461] (molecular function) Definition: Binding to a BLOC-2 complex, a protein complex required for the biogenesis of specialized organelles of the endosomal-lysosomal system, such as melanosomes and platelet dense granules. Relationships: is a type of protein-containing complex binding [GO:0044877] References: PMID:22511774 Sources: GOC:PARL, GOC:bf